{
  "term_label": "Unknown cellular component",
  "gene_symbol": "DNASE2",
  "gene": "UniProtKB:O00115",
  "gene_name": "Deoxyribonuclease-2-alpha",
  "term_id": "UNKNOWN:0003"
}